{
  "gene_symbol": "MDH1B",
  "gene": "UniProtKB:Q5I0G3",
  "term_id": "GO:0019674",
  "term_label": "NAD+ metabolic process",
  "gene_name": "Putative malate dehydrogenase 1B"
}